positive regulation of urea catabolic process [GO:1901714] (biological process) Also known as: activation of urea breakdown, activation of urea catabolism, activation of urea decomposition, activation of urea degradation, positive regulation of urea breakdown, positive regulation of urea catabolism, positive regulation of urea decomposition, positive regulation of urea degradation, up regulation of urea breakdown, up regulation of urea catabolic process, up regulation of urea catabolism, up regulation of urea decomposition, up regulation of urea degradation, up-regulation of urea breakdown, up-regulation of urea catabolic process, up-regulation of urea catabolism, up-regulation of urea decomposition, up-regulation of urea degradation, upregulation of urea breakdown, upregulation of urea catabolic process, upregulation of urea catabolism, upregulation of urea decomposition, upregulation of urea degradation, activation of urea catabolic process Sources: GOC:TermGenie Relationships: is a type of positive regulation of amide catabolic process [GO:0034253]; is a type of regulation of urea catabolic process [GO:0034254]; is a type of positive regulation of small molecule metabolic process [GO:0062013]; is a type of positive regulation of nitrogen cycle metabolic process [GO:1903316]; positively regulates urea catabolic process [GO:0043419] Definition: Any process that activates or increases the frequency, rate or extent of urea catabolic process.